sister chromosome movement towards spindle pole involved in meiotic sister chromatid segregation [GO:0051759] (biological process) Definition: The directed movement of sister chromosomes from the center of the spindle towards the spindle poles, mediated by the shortening of microtubules attached to the chromosomes, during meiosis II. Sources: GOC:ai Relationships: is a type of meiotic chromosome movement towards spindle pole [GO:0016344]; is part of meiotic sister chromatid segregation [GO:0045144] Also known as: meiosis II, sister chromosome movement towards spindle pole, sister chromosome movement towards spindle pole during meiosis II